cardiac neuron development [GO:0060959] (biological process) Relationships: is a type of GO:0048935; is a type of cardiac cell development [GO:0055006]; is part of cardiac neuron differentiation [GO:0060945] Sources: GOC:mtg_heart Also known as: heart neuron development Definition: The process whose specific outcome is the progression of a cardiac neuron over time, from its formation to the mature state.